protein-N-terminal-glutamate acetyltransferase activity [GO:1990190] (molecular function) Relationships: is a type of protein-N-terminal amino-acid acetyltransferase activity [GO:0004596] Also known as: peptide-glutamate-alpha-N-acetyltransferase activity, protein-N-terminal-glutamate-alpha-N-acetyltransferase activity Definition: Catalysis of the reaction: acetyl-CoA + N-terminal L-glutamate in peptide = CoA + N-acetyl-L-glutamate-peptide. References: PMID:23912279 Sources: GOC:al